{
  "gene": "UniProtKB:P20930",
  "gene_name": "Filaggrin",
  "term_label": "establishment of skin barrier",
  "term_id": "GO:0061436",
  "gene_symbol": "FLG"
}